{
  "term_label": "actin filament organization",
  "gene_symbol": "XIRP2",
  "gene": "UniProtKB:A4UGR9",
  "term_id": "GO:0007015",
  "gene_name": "Xin actin-binding repeat-containing protein 2"
}